{
  "gene_name": "Cadherin-1",
  "gene_symbol": "CDH1",
  "term_id": "GO:0043296",
  "term_label": "apical junction complex",
  "gene": "UniProtKB:P12830"
}